anther wall tapetum cell fate specification [GO:0010234] (BP) Also known as: tapetal cell fate specification Relationships: is a type of cell fate specification [GO:0001708]; is a type of developmental process involved in reproduction [GO:0003006]; is part of anther wall tapetum cell differentiation [GO:0048657] Sources: GOC:mg Definition: The process in which a cell becomes capable of differentiating autonomously into a tapetal cell of anthers in an environment that is neutral with respect to the developmental pathway; upon specification, the cell fate can be reversed.